{
  "gene_name": "Inactive phospholipase C-like protein 1",
  "gene": "UniProtKB:Q15111",
  "term_label": "phosphatidylinositol metabolic process",
  "gene_symbol": "PLCL1",
  "term_id": "GO:0046488"
}